{
  "gene_name": "Transmembrane protein 168",
  "gene": "UniProtKB:Q9H0V1",
  "term_label": "Unknown cellular component",
  "term_id": "UNKNOWN:0003",
  "gene_symbol": "TMEM168"
}